{
  "gene_symbol": "GPHN",
  "term_label": "postsynaptic specialization",
  "term_id": "GO:0099572",
  "gene_name": "Gephyrin",
  "gene": "UniProtKB:Q9NQX3"
}